{
  "term_id": "UNKNOWN:0002",
  "term_label": "Unknown biological process",
  "gene_name": "Fibronectin type III and SPRY domain-containing protein 2",
  "gene": "UniProtKB:A1L4K1",
  "gene_symbol": "FSD2"
}